vacuolar sequestering [GO:0043181] (biological process) Sources: GOC:jl Subtypes: vacuolar sequestering of sodium ion [GO:0043182] Also known as: retention in vacuole, sequestering in vacuole, sequestration in vacuole, storage in vacuole, vacuolar retention, vacuolar sequestration, vacuolar storage Relationships: is a type of maintenance of location in cell [GO:0051651] Definition: The process of transporting a substance into, and confining within, a vacuole.